{
  "gene": "UniProtKB:Q9HAW0",
  "gene_name": "Transcription factor IIIB 50 kDa subunit",
  "gene_symbol": "BRF2",
  "term_label": "TBP-class protein binding",
  "term_id": "GO:0017025"
}